{
  "gene_name": "SH3 domain-binding protein 4",
  "gene": "UniProtKB:Q9P0V3",
  "term_id": "UNKNOWN:0002",
  "term_label": "Unknown biological process",
  "gene_symbol": "SH3BP4"
}